{
  "term_id": "UNKNOWN:0002",
  "gene": "UniProtKB:Q8NFV5",
  "gene_symbol": "SPDYE1",
  "term_label": "Unknown biological process",
  "gene_name": "Speedy protein E1"
}